{
  "term_label": "Unknown cellular component",
  "gene_name": "Coiled-coil domain-containing protein 150",
  "gene": "UniProtKB:Q8NCX0",
  "term_id": "UNKNOWN:0003",
  "gene_symbol": "CCDC150"
}